regulation of inhibin secretion [GO:0032338] (biological process) Subtypes: negative regulation of inhibin secretion [GO:0032339], positive regulation of inhibin secretion [GO:0032340] Definition: Any process that modulates the frequency, rate or extent of the regulated release of inhibin from a cell. Relationships: is a type of regulation of endocrine process [GO:0044060]; is a type of regulation of hormone secretion [GO:0046883]; regulates inhibin secretion [GO:0032334] Sources: GOC:mah